positive regulation of astrocyte chemotaxis [GO:2000464] (biological process) Sources: GOC:obol Relationships: is a type of positive regulation of chemotaxis [GO:0050921]; is a type of positive regulation of glial cell migration [GO:1903977]; is a type of regulation of astrocyte chemotaxis [GO:2000458]; positively regulates astrocyte chemotaxis [GO:0035700] Definition: Any process that activates or increases the frequency, rate or extent of astrocyte chemotaxis.